xylotriose transport [GO:2001094] (biological process) Definition: The directed movement of a xylotrioseacetate into, out of or within a cell, or between cells, by means of some agent such as a transporter or pore. Sources: GOC:mengo_curators Relationships: is a type of GO:2001088